{
  "term_id": "GO:0005634",
  "gene": "UniProtKB:Q9UJ98",
  "gene_name": "Cohesin subunit SA-3",
  "term_label": "nucleus",
  "gene_symbol": "STAG3"
}